{
  "gene_symbol": "TRMT13",
  "term_label": "Unknown cellular component",
  "term_id": "UNKNOWN:0003",
  "gene": "UniProtKB:Q9NUP7",
  "gene_name": "tRNA:m(4)X modification enzyme TRM13 homolog"
}